flavonol 7-O-beta-glucosyltransferase activity [GO:0033836] (molecular function) Definition: Catalysis of the reaction: UDP-glucose + a flavonol = UDP + a flavonol 7-O-beta-D-glucoside. Also known as: UDP-glucose:flavonol 7-O-beta-D-glucosyltransferase activity, UDP-glucose:flavonol 7-O-glucosyltransferase activity Sources: EC:2.4.1.237 Relationships: is a type of glucosyltransferase activity [GO:0046527]